{
  "term_label": "aspartic-type endopeptidase activity",
  "gene": "UniProtKB:Q5TDH0",
  "gene_name": "Protein DDI1 homolog 2",
  "gene_symbol": "DDI2",
  "term_id": "GO:0004190"
}